{
  "term_id": "UNKNOWN:0003",
  "gene_symbol": "NIT1",
  "gene_name": "Deaminated glutathione amidase",
  "term_label": "Unknown cellular component",
  "gene": "UniProtKB:Q86X76"
}